{
  "gene_symbol": "SGSM2",
  "term_label": "Unknown cellular component",
  "term_id": "UNKNOWN:0003",
  "gene": "UniProtKB:O43147",
  "gene_name": "Small G protein signaling modulator 2"
}